{
  "term_id": "UNKNOWN:0002",
  "gene_symbol": "RPL27",
  "term_label": "Unknown biological process",
  "gene": "UniProtKB:P61353",
  "gene_name": "Large ribosomal subunit protein eL27"
}